{
  "gene": "UniProtKB:Q9BYM8",
  "gene_name": "RanBP-type and C3HC4-type zinc finger-containing protein 1",
  "gene_symbol": "RBCK1",
  "term_id": "GO:0004842",
  "term_label": "ubiquitin-protein transferase activity"
}